flavone metabolic process [GO:0051552] (biological process) Subtypes: GO:0051553, flavonol metabolic process [GO:0051554], quercetin catabolic process [GO:1901733] Relationships: is a type of flavonoid metabolic process [GO:0009812]; is a type of GO:0042440 References: PMID:18567791 Also known as: flavone metabolism, 2-phenyl-4H-1-benzopyran-4-one metabolic process, 2-phenyl-4H-1-benzopyran-4-one metabolism, 2-phenylchromone metabolic process, 2-phenylchromone metabolism Definition: The chemical reactions and pathways involving flavones, a class of pigmented plant compounds based on 2-phenyl-4H-1-benzopyran-4-one (2-phenylchromone).